regulation of cholesterol efflux [GO:0010874] (biological process) Sources: GOC:BHF, GOC:dph, GOC:tb Subtypes: positive regulation of cholesterol efflux [GO:0010875], negative regulation of cholesterol efflux [GO:0090370] Definition: Any process that modulates the frequency, rate or extent of cholesterol efflux. Cholesterol efflux is the directed movement of cholesterol, cholest-5-en-3-beta-ol, out of a cell or organelle. Relationships: is a type of regulation of cholesterol transport [GO:0032374]; regulates cholesterol efflux [GO:0033344]